tRNA (guanine) methyltransferase activity [GO:0016423] (molecular function) Relationships: is a type of tRNA methyltransferase activity [GO:0008175]; is a type of S-adenosylmethionine-dependent methyltransferase activity [GO:0008757] Subtypes: tRNA (guanine(46)-N7)-methyltransferase activity [GO:0008176], tRNA (guanosine(9)-N1)-methyltransferase activity [GO:0052905], tRNA (guanine(37)-N1)-methyltransferase activity [GO:0052906], tRNA (guanosine(34)-2'-O)-methyltransferase activity [GO:0106340], tRNA (guanine(18)-2'-O)-methyltransferase activity [GO:0141100], GO:0160101, tRNA (guanine(10)-N2)-methyltransferase activity [GO:0160102], tRNA (guanine(26)-N2/guanine(27)-N2)-dimethyltransferase activity [GO:0160103], tRNA (guanine(26)-N2)-dimethyltransferase activity [GO:0160104], GO:0160117, tRNA (guanine(7)-N2)-methyltransferase activity [GO:0160118], GO:0160248 Also known as: tRNA (guanosine) methyltransferase activity Sources: GOC:go-curators Definition: Catalysis of the reaction: S-adenosyl-L-methionine + guanosine in tRNA = S-adenosyl-L-homocysteine + tRNA containing methylguanine.